{
  "term_label": "Unknown molecular function",
  "gene": "UniProtKB:Q8N5G0",
  "gene_name": "Small integral membrane protein 20",
  "term_id": "UNKNOWN:0001",
  "gene_symbol": "SMIM20"
}